{
  "gene": "UniProtKB:A0PJZ3",
  "term_id": "UNKNOWN:0002",
  "gene_name": "Glucoside xylosyltransferase 2",
  "gene_symbol": "GXYLT2",
  "term_label": "Unknown biological process"
}